{
  "gene_symbol": "FNIP1",
  "gene_name": "Folliculin-interacting protein 1",
  "gene": "UniProtKB:Q8TF40",
  "term_label": "protein-folding chaperone binding",
  "term_id": "GO:0051087"
}